{
  "term_label": "cell migration",
  "gene_symbol": "CDH23",
  "gene": "UniProtKB:Q9H251",
  "gene_name": "Cadherin-23",
  "term_id": "GO:0016477"
}